{
  "term_label": "plasma membrane",
  "gene": "UniProtKB:Q9H4L5",
  "term_id": "GO:0005886",
  "gene_name": "Oxysterol-binding protein-related protein 3",
  "gene_symbol": "OSBPL3"
}